{
  "gene": "UniProtKB:Q5VZL5",
  "term_id": "UNKNOWN:0001",
  "gene_name": "Zinc finger MYM-type protein 4",
  "term_label": "Unknown molecular function",
  "gene_symbol": "ZMYM4"
}